positive regulation of miRNA transcription [GO:1902895] (biological process) References: PMID:24699545 Sources: GOC:TermGenie, GOC:dph, GOC:kmv, GO_REF:0000058 Relationships: is a type of GO:0045893; is a type of GO:1902893; is a type of positive regulation of miRNA metabolic process [GO:2000630]; positively regulates GO:0061614 Also known as: positive regulation of microRNA gene transcription, positive regulation of pri-miRNA gene transcription, positive regulation of pri-miRNA transcription by RNA polymerase II, positive regulation of pri-miRNA transcription from RNA polymerase II promoter, positive regulation of primary miRNA gene transcription, up regulation of pri-miRNA transcription from RNA polymerase II promoter, up-regulation of pri-miRNA transcription from RNA polymerase II promoter, upregulation of pri-miRNA transcription from RNA polymerase II promoter, activation of pri-miRNA transcription from RNA polymerase II promoter Definition: Any process that activates or increases the frequency, rate or extent of microRNA (miRNA) gene transcription.